positive regulation of arugosin biosynthetic process [GO:1900628] (biological process) Definition: Any process that activates or increases the frequency, rate or extent of arugosin biosynthetic process. Relationships: is a type of GO:1900378; is a type of regulation of arugosin biosynthetic process [GO:1900626]; positively regulates arugosin biosynthetic process [GO:1900587] Also known as: activation of arugosin anabolism, activation of arugosin biosynthesis, activation of arugosin formation, activation of arugosin synthesis, positive regulation of arugosin anabolism, positive regulation of arugosin biosynthesis, positive regulation of arugosin formation, positive regulation of arugosin synthesis, up regulation of arugosin anabolism, up regulation of arugosin biosynthesis, up regulation of arugosin biosynthetic process, up regulation of arugosin formation, up regulation of arugosin synthesis, up-regulation of arugosin anabolism, up-regulation of arugosin biosynthesis, up-regulation of arugosin biosynthetic process, up-regulation of arugosin formation, up-regulation of arugosin synthesis, upregulation of arugosin anabolism, upregulation of arugosin biosynthesis, upregulation of arugosin biosynthetic process, upregulation of arugosin formation, upregulation of arugosin synthesis, activation of arugosin biosynthetic process Sources: GOC:TermGenie, GOC:di